1-deoxy-D-xylulose-5-phosphate synthase activity [GO:0008661] (molecular function) Also known as: 1-deoxy-D-xylulose-5-phosphate pyruvate-lyase (carboxylating) activity, 1-deoxyxylulose-5-phosphate synthase activity, DOXP synthase activity, DXP-synthase activity, pyruvate:D-glyceraldehyde-3-phosphate acetaldehydetransferase (decarboxylating) Sources: EC:2.2.1.7, RHEA:12605 Relationships: is a type of transketolase or transaldolase activity [GO:0016744] Definition: Catalysis of the reaction: D-glyceraldehyde 3-phosphate + H+ + pyruvate = 1-deoxy-D-xylulose 5-phosphate + CO2.